specification of segmental identity, thorax [GO:0007384] (biological process) Sources: ISBN:0878932437 Relationships: is a type of specification of segmental identity, trunk [GO:0035292] Definition: The specification of the characteristic structures of the thoracic segments following establishment of segment boundaries. Identity is considered to be the aggregate of characteristics by which a structure is recognized.